response to epinephrine [GO:0071871] (biological process) Subtypes: GO:0071872 Definition: Any process that results in a change in state or activity of a cell or an organism (in terms of movement, secretion, enzyme production, gene expression, etc.) as a result of an epinephrine stimulus. Epinephrine is a catecholamine that has the formula C9H13NO3; it is secreted by the adrenal medulla to act as a hormone, and released by certain neurons to act as a neurotransmitter active in the central nervous system. Relationships: is a type of response to chemical [GO:0042221] Sources: GOC:BHF, GOC:mah Also known as: response to adrenaline stimulus, response to epinephrine stimulus Note: Note that epinephrine and norepinephrine are ligands for the same receptors, and there are multiple adrenergic receptors.